positive regulation of T cell extravasation [GO:2000409] (biological process) Relationships: is a type of positive regulation of cellular extravasation [GO:0002693]; is a type of positive regulation of T cell migration [GO:2000406]; is a type of GO:2000407; positively regulates GO:0072683 Definition: Any process that activates or increases the frequency, rate or extent of T cell extravasation. Also known as: positive regulation of T lymphocyte extravasation, positive regulation of T-cell extravasation, positive regulation of T-lymphocyte extravasation Subtypes: positive regulation of CD8-positive, alpha-beta T cell extravasation [GO:2000451] Sources: GOC:BHF, GOC:mah